galactosyl beta-1,3 N-acetylgalactosamine beta-1,3-glucuronosyltransferase activity [GO:0046989] (molecular function) Definition: Catalysis of the transfer, in a beta 1,3 linkage, of D-glucuronic acid (GlcUA) from UDP-GlcUA to the disaccharide galactosyl beta-1,3 N-acetylgalactosamine, a common component of glycoproteins and glycolipids. References: PMID:12511570 Sources: GOC:bf Relationships: is_a glucuronosyltransferase activity [GO:0015020]